positive regulation of dendritic spine development [GO:0060999] (biological process) Subtypes: positive regulation of dendritic spine morphogenesis [GO:0061003] Sources: GOC:dph Relationships: is a type of positive regulation of developmental process [GO:0051094]; is a type of regulation of dendritic spine development [GO:0060998]; RO_0002213 dendritic spine development [GO:0060996] Definition: Any process that increases the rate, frequency, or extent of dendritic spine development, the process whose specific outcome is the progression of the dendritic spine over time, from its formation to the mature structure.